{
  "gene_name": "Dolichyl-diphosphooligosaccharide--protein glycosyltransferase subunit 4",
  "gene_symbol": "OST4",
  "gene": "UniProtKB:P0C6T2",
  "term_id": "GO:0008250",
  "term_label": "oligosaccharyltransferase complex"
}